{
  "term_id": "GO:0006308",
  "gene_name": "Deoxyribonuclease-1-like 1",
  "gene_symbol": "DNASE1L1",
  "term_label": "DNA catabolic process",
  "gene": "UniProtKB:P49184"
}